{
  "term_label": "RISC complex",
  "term_id": "GO:0016442",
  "gene_symbol": "AGO3",
  "gene": "UniProtKB:Q9H9G7",
  "gene_name": "Protein argonaute-3"
}